THO complex [GO:0000347] (cellular component) References: PMID:11060033, PMID:11979277, PMID:16983072 Sources: GOC:krc Relationships: is_a nuclear protein-containing complex [GO:0140513] Definition: The THO complex is a nuclear complex that is required for transcription elongation through genes containing tandemly repeated DNA sequences. The THO complex is also part of the TREX (TRanscription EXport) complex that is involved in coupling transcription to export of mRNAs to the cytoplasm. In S. cerevisiae, it is composed of four subunits: Hpr1p, Tho2p, Thp1p, and Mft1p, while the human complex is composed of 7 subunits. Subtypes: GO:0000445, nucleoplasmic THO complex [GO:0000446]